{
  "term_id": "GO:0034451",
  "term_label": "centriolar satellite",
  "gene_symbol": "PCM1",
  "gene": "UniProtKB:Q15154",
  "gene_name": "Pericentriolar material 1 protein"
}